{
  "gene_name": "Src kinase-associated phosphoprotein 2",
  "gene_symbol": "SKAP2",
  "term_label": "plasma membrane",
  "gene": "UniProtKB:O75563",
  "term_id": "GO:0005886"
}